interneuron migration [GO:1904936] (biological process) References: PMID:18622031 Sources: GOC:TermGenie, GOC:ah, GO_REF:0000091 Also known as: inter neuron migration, inter-neuron migration Relationships: is a type of neuron migration [GO:0001764] Subtypes: GO:0021853 Definition: The orderly movement of an interneuron from one site to another.